{
  "gene": "UniProtKB:Q4V339",
  "term_label": "zinc ion binding",
  "gene_name": "Zinc-regulated GTPase metalloprotein activator 1F",
  "term_id": "GO:0008270",
  "gene_symbol": "ZNG1F"
}